{
  "term_label": "histone H3K9 demethylase activity",
  "gene_name": "Lysine-specific demethylase 4E",
  "gene": "UniProtKB:B2RXH2",
  "term_id": "GO:0032454",
  "gene_symbol": "KDM4E"
}